{
  "gene_symbol": "TSPAN13",
  "gene_name": "Tetraspanin-13",
  "term_id": "UNKNOWN:0001",
  "term_label": "Unknown molecular function",
  "gene": "UniProtKB:O95857"
}